{
  "gene": "UniProtKB:O00327",
  "term_label": "aryl hydrocarbon receptor complex",
  "term_id": "GO:0034751",
  "gene_symbol": "BMAL1",
  "gene_name": "Basic helix-loop-helix ARNT-like protein 1"
}